single-stranded DNA binding [GO:0003697] (molecular function) Also known as: ssDNA binding Subtypes: sequence-specific single stranded DNA binding [GO:0098847], DNA/DNA annealing activity [GO:1990814], C-rich single-stranded DNA binding [GO:1990829], G-rich single-stranded DNA binding [GO:1990955] References: PMID:22976174 Sources: GOC:elh, GOC:vw Definition: Binding to single-stranded DNA. Relationships: is a type of DNA binding [GO:0003677] Note: Note that this term is restricted to those cases where the binding is to a single-stranded DNA molecule, not to one of the stands of double-stranded DNA.